regulation of sperm capacitation [GO:1902490] (biological process) Definition: Any process that modulates the frequency, rate or extent of sperm capacitation. Subtypes: negative regulation of sperm capacitation [GO:1902491], GO:1902492 References: PMID:22539676 Sources: GOC:TermGenie, GOC:hjd Relationships: is a type of GO:0051239; is a type of regulation of cell maturation [GO:1903429]; is a type of regulation of reproductive process [GO:2000241]; regulates sperm capacitation [GO:0048240] Also known as: regulation of sperm activation